{
  "term_label": "fat cell differentiation",
  "term_id": "GO:0045444",
  "gene_name": "Constitutive coactivator of peroxisome proliferator-activated receptor gamma",
  "gene": "UniProtKB:Q96EK7",
  "gene_symbol": "FAM120B"
}